{
  "gene_name": "Leucine-rich repeat-containing protein 47",
  "term_id": "UNKNOWN:0003",
  "gene": "UniProtKB:Q8N1G4",
  "gene_symbol": "LRRC47",
  "term_label": "Unknown cellular component"
}